{
  "term_label": "Unknown biological process",
  "gene": "UniProtKB:O15225",
  "gene_name": "Putative inactivation escape 1 protein",
  "gene_symbol": "INE1",
  "term_id": "UNKNOWN:0002"
}